{
  "term_label": "Unknown molecular function",
  "gene_name": "Putative uncharacterized protein KIRREL3-AS3",
  "term_id": "UNKNOWN:0001",
  "gene_symbol": "KIRREL3-AS3",
  "gene": "UniProtKB:Q8N7Y1"
}